{
  "gene_name": "Long-chain specific acyl-CoA dehydrogenase, mitochondrial",
  "gene": "UniProtKB:P28330",
  "term_label": "long-chain fatty acyl-CoA dehydrogenase activity",
  "term_id": "GO:0004466",
  "gene_symbol": "ACADL"
}